{
  "term_label": "Unknown cellular component",
  "gene_name": "Putative uncharacterized protein BVES-AS1",
  "gene": "UniProtKB:Q5T3Y7",
  "term_id": "UNKNOWN:0003",
  "gene_symbol": "BVES-AS1"
}